{
  "gene": "UniProtKB:P11413",
  "term_id": "GO:0009051",
  "gene_symbol": "G6PD",
  "term_label": "pentose-phosphate shunt, oxidative branch",
  "gene_name": "Glucose-6-phosphate 1-dehydrogenase"
}